positive regulation of apical ectodermal ridge formation [GO:1905142] (biological process) Definition: Any process that activates or increases the frequency, rate or extent of apical ectodermal ridge formation. Also known as: positive regulation of apical epidermal ridge formation, up regulation of apical ectodermal ridge formation, up regulation of apical epidermal ridge formation, up-regulation of apical ectodermal ridge formation, up-regulation of apical epidermal ridge formation, upregulation of apical ectodermal ridge formation, upregulation of apical epidermal ridge formation, activation of AER formation, positive regulation of AER formation, positive regulation of crista ectodermalis apicalis formation, up regulation of AER formation, up regulation of crista ectodermalis apicalis formation, up-regulation of AER formation, up-regulation of crista ectodermalis apicalis formation, upregulation of AER formation, upregulation of crista ectodermalis apicalis formation Relationships: is a type of GO:0051094; is a type of positive regulation of multicellular organismal process [GO:0051240]; is a type of regulation of apical ectodermal ridge formation [GO:1905140]; positively regulates apical ectodermal ridge formation [GO:1905139] References: PMID:18359901 Sources: GOC:TermGenie, GO_REF:0000058